{
  "term_label": "cilium assembly",
  "gene_name": "Protein inturned",
  "gene": "UniProtKB:Q9ULD6",
  "gene_symbol": "INTU",
  "term_id": "GO:0060271"
}